cellular response to fructose stimulus [GO:0071332] (biological process) Sources: GOC:mah Relationships: is a type of response to fructose [GO:0009750]; is a type of GO:0071331 Definition: Any process that results in a change in state or activity of a cell (in terms of movement, secretion, enzyme production, gene expression, etc.) as a result of a fructose stimulus.